{
  "gene_name": "Ras-related protein Rab-17",
  "gene": "UniProtKB:Q9H0T7",
  "term_id": "GO:0055038",
  "gene_symbol": "RAB17",
  "term_label": "recycling endosome membrane"
}